{
  "term_id": "GO:0045041",
  "gene_symbol": "CHCHD4",
  "gene": "UniProtKB:Q8N4Q1",
  "gene_name": "Mitochondrial intermembrane space import and assembly protein 40",
  "term_label": "protein import into mitochondrial intermembrane space"
}